{
  "term_label": "extracellular matrix",
  "gene_symbol": "LTBP1",
  "term_id": "GO:0031012",
  "gene_name": "Latent-transforming growth factor beta-binding protein 1",
  "gene": "UniProtKB:Q14766"
}